{
  "gene": "UniProtKB:Q69YI7",
  "term_label": "Unknown molecular function",
  "gene_name": "Nuclear apoptosis-inducing factor 1",
  "term_id": "UNKNOWN:0001",
  "gene_symbol": "NAIF1"
}